mannosyl-3-phosphoglycerate synthase activity [GO:0050504] (molecular function) Definition: Catalysis of the reaction: 3-phospho-D-glycerate + GDP-alpha-D-mannose = 2-(alpha-D-mannosyl)-3-phosphoglycerate + GDP + H+. Relationships: is_a hexosyltransferase activity [GO:0016758] Sources: EC:2.4.1.217, RHEA:13537 Also known as: GDP-mannose:3-phosphoglycerate 3-alpha-D-mannosyltransferase activity, MPG synthase activity